mitochondrial outer membrane fusion [GO:1990626] (BP) Relationships: is a type of outer mitochondrial membrane organization [GO:0007008]; BFO_0000050 mitochondrial fusion [GO:0008053] References: PMID:21385840 Sources: GOC:vw Also known as: mitochondrion outer membrane fusion Definition: The membrane organization process that joins two mitochondrial outer membranes to form a single membrane.